{
  "gene_symbol": "MRPL15",
  "gene": "UniProtKB:Q9P015",
  "term_id": "GO:0005762",
  "term_label": "mitochondrial large ribosomal subunit",
  "gene_name": "Large ribosomal subunit protein uL15m"
}